{
  "gene_symbol": "LAMP5",
  "gene_name": "Lysosome-associated membrane glycoprotein 5",
  "term_label": "Unknown molecular function",
  "term_id": "UNKNOWN:0001",
  "gene": "UniProtKB:Q9UJQ1"
}